{
  "gene_symbol": "EXOC6",
  "gene": "UniProtKB:Q8TAG9",
  "term_label": "exocyst",
  "term_id": "GO:0000145",
  "gene_name": "Exocyst complex component 6"
}